{
  "term_id": "GO:0016485",
  "term_label": "protein processing",
  "gene_name": "Nicastrin",
  "gene_symbol": "NCSTN",
  "gene": "UniProtKB:Q92542"
}